vitamin B6 catabolic process [GO:0042820] (biological process) References: PMID:30037155, PMID:30671974 Sources: GOC:jl Relationships: is a type of water-soluble vitamin catabolic process [GO:0042365]; is a type of GO:0042816; is a type of pyridine-containing compound catabolic process [GO:0072526] Also known as: vitamin B6 breakdown, vitamin B6 catabolism, vitamin B6 degradation Definition: The chemical reactions and pathways resulting in the breakdown of any of the vitamin B6 compounds; pyridoxal, pyridoxamine and pyridoxine and the active form, pyridoxal phosphate. Subtypes: pyridoxal phosphate catabolic process [GO:0032361]